{
  "term_id": "GO:0032486",
  "gene": "UniProtKB:P61224",
  "gene_symbol": "RAP1B",
  "gene_name": "Ras-related protein Rap-1b",
  "term_label": "Rap protein signal transduction"
}